positive regulation of male pigmentation [GO:0048093] (biological process) Definition: Any process that activates or increases the frequency, rate or extent of establishment of a pattern of pigment in males. Relationships: is a type of positive regulation of developmental pigmentation [GO:0048087]; is a type of GO:0048088; is a type of positive regulation of developmental process [GO:0051094]; is a type of positive regulation of multicellular organismal process [GO:0051240]; is a type of positive regulation of reproductive process [GO:2000243]; RO_0002213 GO:0048094 Also known as: up regulation of male pigmentation, up-regulation of male pigmentation, upregulation of male pigmentation, activation of male pigmentation, stimulation of male pigmentation Sources: GOC:jid